{
  "gene_symbol": "CLDN19",
  "term_id": "GO:0003406",
  "gene": "UniProtKB:Q8N6F1",
  "term_label": "retinal pigment epithelium development",
  "gene_name": "Claudin-19"
}